{
  "gene": "UniProtKB:Q8TBA6",
  "term_label": "Golgi cisterna",
  "gene_name": "Golgin subfamily A member 5",
  "gene_symbol": "GOLGA5",
  "term_id": "GO:0031985"
}